caste determination, influence by genetic factors [GO:0048649] (biological process) Definition: The process in which individuals, having the potential to develop any of several distinct developmental paths, have their individual developmental fate determined in response to genetic cues. Individuals with distinct developmental fates perform different functions in a colony of social insects. Relationships: is_a caste determination [GO:0048648]; is a type of GO:0048652 Sources: GOC:jid